propanediol degradation polyhedral organelle [GO:0031472] (cellular component) References: PMID:10498708, PMID:11844753, PMID:12923081 Sources: GOC:js Definition: An organelle found in bacteria consisting of a proteinaceous coat containing enzymes for the degradation of 1,2-propanediol whose purpose is the protection of the rest of the cell from the toxic propionaldehyde product of the enzyme diol dehydratase. Relationships: is a type of bacterial microcompartment [GO:0031469]